{
  "term_id": "UNKNOWN:0002",
  "gene_name": "Uncharacterized protein FLJ40521",
  "term_label": "Unknown biological process",
  "gene": "UniProtKB:Q8N7P7",
  "gene_symbol": "Q8N7P7"
}